{
  "term_label": "chloride:bicarbonate antiporter activity",
  "gene": "UniProtKB:Q7LBE3",
  "gene_symbol": "SLC26A9",
  "gene_name": "Solute carrier family 26 member 9",
  "term_id": "GO:0140900"
}